{
  "term_label": "regulation of transcription by RNA polymerase II",
  "gene_name": "Zinc finger protein 184",
  "term_id": "GO:0006357",
  "gene_symbol": "ZNF184",
  "gene": "UniProtKB:Q99676"
}